{
  "gene_name": "NACHT, LRR and PYD domains-containing protein 8",
  "term_id": "GO:0050727",
  "gene_symbol": "NLRP8",
  "gene": "UniProtKB:Q86W28",
  "term_label": "regulation of inflammatory response"
}